epidermal lamellar body membrane [GO:0097234] (cellular component) Relationships: is a type of GO:0097232; is part of GO:0097209 References: PMID:11940594 Sources: GOC:sl Definition: The lipid bilayer surrounding an epidermal lamellar body, a specialized secretory organelle found in keratinocytes and involved in the formation of an impermeable, lipid-containing membrane that serves as a water barrier and is required for correct skin barrier function.